cell cycle process [GO:0022402] (biological process) Relationships: is a type of GO:0009987; BFO_0000050 cell cycle [GO:0007049] Subtypes: re-entry into mitotic cell cycle [GO:0000320], cytokinesis [GO:0000910], preprophase band assembly [GO:0000913], cell plate assembly [GO:0000919], spindle organization [GO:0007051], chromosome segregation [GO:0007059], GO:0007062, GO:0007098, centriole replication [GO:0007099], regulation of syncytial blastoderm mitotic cell cycle [GO:0007348], attachment of spindle microtubules to kinetochore [GO:0008608], centriole-centriole cohesion [GO:0010457], telomere maintenance via semi-conservative replication [GO:0032201], cytokinetic process [GO:0032506], GO:0034085, maintenance of sister chromatid cohesion [GO:0034086], centromere separation [GO:0034510], microtubule anchoring at spindle pole body [GO:0034631], GO:0044770, GO:0044786, actomyosin contractile ring organization [GO:0044837], G0 to G1 transition [GO:0045023], spindle elongation [GO:0051231], GO:0051255, centrosome duplication [GO:0051298], centrosome separation [GO:0051299], spindle pole body organization [GO:0051300], chromosome separation [GO:0051304], chromosome movement towards spindle pole [GO:0051305], spindle localization [GO:0051653], cell cycle switching [GO:0060184], centriole elongation [GO:0061511], G1 to G0 transition [GO:0070314], DNA replication preinitiation complex assembly [GO:0071163], GO:0071990, GO:0090399, chromosome attachment to the nuclear envelope [GO:0097240], spindle pole body separation [GO:0110100], repair of kinetochore microtubule attachment defect [GO:0140274], MCM complex loading [GO:0140530], cell cycle DNA replication initiation [GO:1902292], cell cycle DNA replication termination [GO:1902294], DNA strand elongation involved in cell cycle DNA replication [GO:1902296], GO:1902298, pre-replicative complex assembly involved in cell cycle DNA replication [GO:1902299], meiotic cell cycle process [GO:1903046], mitotic cell cycle process [GO:1903047], actomyosin contractile ring assembly actin filament organization [GO:2000689] Sources: GOC:isa_complete, GOC:mtg_cell_cycle Regulation: regulated by GO:0010564; negatively regulated by GO:0010948; positively regulated by positive regulation of cell cycle process [GO:0090068] Definition: The cellular process that ensures successive accurate and complete genome replication and chromosome segregation.